{
  "gene": "UniProtKB:P54317",
  "gene_name": "Pancreatic lipase-related protein 2",
  "gene_symbol": "PNLIPRP2",
  "term_label": "phospholipase A1 activity",
  "term_id": "GO:0008970"
}